{
  "term_label": "keratinization",
  "gene": "UniProtKB:Q7RTS7",
  "term_id": "GO:0031424",
  "gene_name": "Keratin, type II cytoskeletal 74",
  "gene_symbol": "KRT74"
}